N-acetyl-L-aspartate-L-glutamate ligase activity [GO:0072590] (molecular function) References: PMID:20643647, PMID:20657015 Definition: Catalysis of the reaction: ATP + N-acetyl-L-aspartate + L-glutamate = ADP + phosphate + N-acetylaspartyl-glutamate. Relationships: is a type of ligase activity, forming carbon-nitrogen bonds [GO:0016879]